{
  "term_label": "intracellular protein transport",
  "term_id": "GO:0006886",
  "gene_name": "Vacuolar protein sorting-associated protein 29",
  "gene_symbol": "VPS29",
  "gene": "UniProtKB:Q9UBQ0"
}